{
  "gene_symbol": "TUBGCP6",
  "term_label": "gamma-tubulin binding",
  "gene": "UniProtKB:Q96RT7",
  "gene_name": "Gamma-tubulin complex component 6",
  "term_id": "GO:0043015"
}